{
  "term_id": "GO:0000502",
  "gene_name": "Putative protein SEM1, isoform 2",
  "term_label": "proteasome complex",
  "gene_symbol": "SEM1",
  "gene": "UniProtKB:Q6ZVN7"
}